{
  "term_label": "Unknown cellular component",
  "gene": "UniProtKB:A0A0J9YY99",
  "gene_name": "Ig-like domain-containing protein (Fragment)",
  "term_id": "UNKNOWN:0003",
  "gene_symbol": "A0A0J9YY99"
}